{
  "gene_symbol": "RNF138",
  "gene": "UniProtKB:Q8WVD3",
  "gene_name": "E3 ubiquitin-protein ligase RNF138",
  "term_id": "GO:0010792",
  "term_label": "DNA double-strand break processing involved in repair via single-strand annealing"
}